{
  "gene_symbol": "DNAH14",
  "gene": "UniProtKB:Q0VDD8",
  "term_label": "minus-end-directed microtubule motor activity",
  "gene_name": "Dynein axonemal heavy chain 14",
  "term_id": "GO:0008569"
}